{
  "gene_symbol": "FGF18",
  "gene_name": "Fibroblast growth factor 18",
  "term_id": "GO:0022008",
  "term_label": "neurogenesis",
  "gene": "UniProtKB:O76093"
}